{
  "gene": "UniProtKB:Q9H902",
  "gene_symbol": "REEP1",
  "term_label": "endoplasmic reticulum tubular network organization",
  "gene_name": "Receptor expression-enhancing protein 1",
  "term_id": "GO:0071786"
}